detection of mechanical stimulus involved in sensory perception [GO:0050974] (biological process) Sources: GOC:ai, GOC:dos Also known as: sensory detection of mechanical stimulus, sensory detection of mechanical stimulus during sensory perception, sensory perception, sensory detection of mechanical stimulus, sensory perception, sensory transduction of mechanical stimulus, sensory transduction of mechanical stimulus, sensory transduction of mechanical stimulus during sensory perception Definition: The series of events in which a mechanical stimulus is received and converted into a molecular signal as part of sensory perception. Subtypes: detection of mechanical stimulus involved in sensory perception of sound [GO:0050910], detection of mechanical stimulus involved in sensory perception of pain [GO:0050966], detection of mechanical stimulus involved in magnetoreception [GO:0050971], detection of mechanical stimulus involved in echolocation [GO:0050972], detection of mechanical stimulus involved in equilibrioception [GO:0050973], detection of mechanical stimulus involved in sensory perception of touch [GO:0050976], GO:0070999, detection of mechanical stimulus involved in sensory perception of wind [GO:0071066] Relationships: is a type of detection of stimulus involved in sensory perception [GO:0050906]; is a type of detection of mechanical stimulus [GO:0050982]; is part of GO:0050954